{
  "term_label": "receptor complex",
  "gene": "UniProtKB:Q14627",
  "gene_name": "Interleukin-13 receptor subunit alpha-2",
  "gene_symbol": "IL13RA2",
  "term_id": "GO:0043235"
}